{
  "term_id": "GO:0031594",
  "gene": "UniProtKB:Q13702",
  "term_label": "neuromuscular junction",
  "gene_name": "43 kDa receptor-associated protein of the synapse",
  "gene_symbol": "RAPSN"
}